positive regulation of RNA import into nucleus [GO:0046830] (biological process) Definition: Any process that activates or increases the frequency, rate or extent of movement of RNA from the cytoplasm into the nucleus. Also known as: positive regulation of RNA import into cell nucleus, positive regulation of RNA transport from cytoplasm to nucleus, positive regulation of RNA-nucleus import, up regulation of RNA import into nucleus, up-regulation of RNA import into nucleus, upregulation of RNA import into nucleus, activation of RNA import into nucleus, stimulation of RNA import into nucleus Sources: GOC:bf Relationships: is a type of positive regulation of nucleobase-containing compound transport [GO:0032241]; is_a positive regulation of nucleocytoplasmic transport [GO:0046824]; is_a regulation of RNA import into nucleus [GO:0046828]; positively regulates RNA import into nucleus [GO:0006404]